regulation of skeletal muscle contraction [GO:0014819] (BP) Sources: GOC:ef, GOC:mtg_muscle Subtypes: regulation of skeletal muscle contraction by calcium ion signaling [GO:0014722], regulation of twitch skeletal muscle contraction [GO:0014724], regulation of tonic skeletal muscle contraction [GO:0014746], regulation of skeletal muscle contraction by neural stimulation via neuromuscular junction [GO:0014852], GO:0014861, regulation of skeletal muscle contraction by chemo-mechanical energy conversion [GO:0014862], regulation of skeletal muscle contraction by action potential [GO:0100001] Definition: Any process that modulates the frequency, rate or extent of skeletal muscle contraction. Relationships: is a type of regulation of striated muscle contraction [GO:0006942]; regulates skeletal muscle contraction [GO:0003009]